positive regulation of inner ear auditory receptor cell differentiation [GO:0045609] (biological process) Sources: GOC:go_curators Relationships: is a type of GO:0045606; is a type of regulation of inner ear auditory receptor cell differentiation [GO:0045607]; is a type of positive regulation of inner ear receptor cell differentiation [GO:2000982]; positively regulates inner ear auditory receptor cell differentiation [GO:0042491] Also known as: positive regulation of auditory hair cell differentiation, up regulation of auditory receptor cell differentiation, up-regulation of auditory receptor cell differentiation, upregulation of auditory receptor cell differentiation, activation of auditory receptor cell differentiation, stimulation of auditory receptor cell differentiation, positive regulation of auditory receptor cell differentiation Definition: Any process that activates or increases the frequency, rate or extent of auditory hair cell differentiation.